{
  "gene": "UniProtKB:Q8WTS6",
  "term_id": "GO:0070828",
  "term_label": "heterochromatin organization",
  "gene_name": "Histone-lysine N-methyltransferase SETD7",
  "gene_symbol": "SETD7"
}